negative regulation of calcineurin-mediated signaling [GO:0106057] (biological process) Relationships: is a type of GO:0050849; is a type of regulation of calcineurin-mediated signaling [GO:0106056]; negatively regulates calcineurin-mediated signaling [GO:0097720] Definition: Any process that stops, prevents or reduces the frequency, rate or extent of calcineurin-mediated signaling. Subtypes: negative regulation of calcineurin-NFAT signaling cascade [GO:0070885] References: PMID:25081204